{
  "gene": "UniProtKB:P30531",
  "gene_symbol": "SLC6A1",
  "term_id": "GO:0005332",
  "gene_name": "Sodium- and chloride-dependent GABA transporter 1",
  "term_label": "gamma-aminobutyric acid:sodium:chloride symporter activity"
}